{
  "term_id": "UNKNOWN:0003",
  "gene": "UniProtKB:Q15027",
  "term_label": "Unknown cellular component",
  "gene_symbol": "ACAP1",
  "gene_name": "Arf-GAP with coiled-coil, ANK repeat and PH domain-containing protein 1"
}